positive regulation of axon guidance [GO:1902669] (BP) References: PMID:23006775 Sources: GOC:TermGenie, GOC:hjd, GO_REF:0000058 Relationships: is a type of positive regulation of neuron projection development [GO:0010976]; is a type of regulation of axon guidance [GO:1902667]; positively regulates axon guidance [GO:0007411] Also known as: positive regulation of axon pathfinding, up regulation of axon guidance, up regulation of axon pathfinding, up-regulation of axon guidance, up-regulation of axon pathfinding, upregulation of axon guidance, upregulation of axon pathfinding, activation of axon growth cone guidance, activation of axon guidance, activation of axon pathfinding, positive regulation of axon growth cone guidance, up regulation of axon growth cone guidance, up-regulation of axon growth cone guidance, upregulation of axon growth cone guidance, activation of axon chemotaxis, positive regulation of axon chemotaxis, up regulation of axon chemotaxis, up-regulation of axon chemotaxis, upregulation of axon chemotaxis Definition: Any process that activates or increases the frequency, rate or extent of axon guidance. Subtypes: positive regulation of retinal ganglion cell axon guidance [GO:1902336], positive regulation of anterior/posterior axon guidance [GO:1905488], positive regulation of sensory neuron axon guidance [GO:1905491], GO:1905814, GO:1905817